{
  "term_id": "GO:0003713",
  "gene_symbol": "PPARGC1A",
  "gene": "UniProtKB:Q9UBK2",
  "gene_name": "Peroxisome proliferator-activated receptor gamma coactivator 1-alpha",
  "term_label": "transcription coactivator activity"
}